{
  "gene": "UniProtKB:P35398",
  "gene_symbol": "RORA",
  "gene_name": "Nuclear receptor ROR-alpha",
  "term_label": "oxysterol binding",
  "term_id": "GO:0008142"
}